dol-P-Man:Man(2)GlcN-acyl-PI alpha-1,2-mannosyltransferase activity [GO:0120564] (molecular function) Relationships: is a type of alpha-1,2-mannosyltransferase activity [GO:0000026]; is_a GPI mannosyltransferase activity [GO:0004376] Definition: Catalysis of the transfer of an alpha-D-mannosyl residue from dolichol-P-mannose to Man(2)-GlcN-acyl-PI, forming an alpha-(1->2)-D-mannosyl-D-mannose linkage. This transfers the third mannose to the GPI precursor. References: PMID:8861954 Also known as: GPI-MT-III activity, glycosylphosphatidylinositol-mannosyltransferase III activity